hyphal membrane [GO:0085039] (cellular component) Definition: A host-derived membrane surrounding the symbiont hypha during infection. Sources: GOC:pamgo_curators Also known as: extra-invasive hyphal membrane Relationships: is a type of host cell membrane [GO:0033644]